transferase activity [GO:0016740] (MF) Definition: Catalysis of the transfer of a group, e.g. a methyl group, glycosyl group, acyl group, phosphorus-containing, or other groups, from one compound (generally regarded as the donor) to another compound (generally regarded as the acceptor). Transferase is the systematic name for any enzyme of EC class 2. Sources: EC:2.-.-.- Relationships: is a type of GO:0003824 Subtypes: GO:0010280, transferase activity, transferring one-carbon groups [GO:0016741], transketolase or transaldolase activity [GO:0016744], acyltransferase activity [GO:0016746], GO:0016757, transferase activity, transferring alkyl or aryl (other than methyl) groups [GO:0016765], transferase activity, transferring nitrogenous groups [GO:0016769], transferase activity, transferring phosphorus-containing groups [GO:0016772], transferase activity, transferring sulphur-containing groups [GO:0016782], selenotransferase activity [GO:0016785], glucanosyltransferase activity [GO:0042123], GO:0061599, microtubule plus end polymerase [GO:0061863], THPH synthase activity [GO:0106265], 4-amino-5-hydroxymethyl-2-methylpyrimidine phosphate synthase activity from histidine and PLP [GO:0106344], GO:0140853, tRNA 5-taurinomethyluridine synthase activity [GO:0160236] Regulation: regulated by regulation of transferase activity [GO:0051338]